{
  "gene_symbol": "STAG1",
  "gene_name": "Cohesin subunit SA-1",
  "term_id": "GO:0000785",
  "gene": "UniProtKB:Q8WVM7",
  "term_label": "chromatin"
}